{
  "term_id": "GO:0007156",
  "gene_symbol": "CEACAM8",
  "gene_name": "Carcinoembryonic antigen-related cell adhesion molecule 8",
  "gene": "UniProtKB:P31997",
  "term_label": "homophilic cell-cell adhesion"
}